{
  "term_label": "Unknown biological process",
  "term_id": "UNKNOWN:0002",
  "gene_name": "eEF1A lysine and N-terminal methyltransferase",
  "gene": "UniProtKB:Q8N6R0",
  "gene_symbol": "METTL13"
}